regulation of blood vessel endothelial cell migration [GO:0043535] (biological process) Definition: Any process that modulates the frequency, rate or extent of the migration of the endothelial cells of blood vessels. Sources: GOC:go_curators Relationships: is a type of GO:0010594; RO_0002211 blood vessel endothelial cell migration [GO:0043534] Subtypes: positive regulation of blood vessel endothelial cell migration [GO:0043536], GO:0043537, GO:0090049